{
  "gene_name": "E3 ubiquitin-protein ligase CHIP",
  "term_id": "GO:0045862",
  "gene_symbol": "STUB1",
  "gene": "UniProtKB:Q9UNE7",
  "term_label": "positive regulation of proteolysis"
}